thiamine pyrophosphate transmembrane transport [GO:0030974] (BP) Subtypes: mitochondrial thiamine pyrophosphate transmembrane transport [GO:1990545] Also known as: TPP transport, thiamin diphosphate transport, thiamin pyrophosphate transport, thiamine diphosphate transport, thiamine pyrophosphate transport Sources: GOC:mlg Relationships: is a type of quaternary ammonium group transport [GO:0015697]; is a type of organic anion transport [GO:0015711]; is_a organophosphate ester transport [GO:0015748]; is a type of thiamine transmembrane transport [GO:0071934] Definition: The process in which thiamine pyrophosphate is transported across a membrane.